{
  "gene": "UniProtKB:Q8N412",
  "term_label": "Unknown molecular function",
  "gene_name": "Sperm-tail PG-rich repeat-containing protein 2",
  "gene_symbol": "STPG2",
  "term_id": "UNKNOWN:0001"
}